enzyme-directed rRNA pseudouridine synthesis [GO:0000455] (biological process) Definition: The intramolecular conversion of uridine to pseudouridine during ribosome biogenesis where the enzyme specifies the site that becomes pseudouridylated without using a guide RNA. Sources: GOC:curators, ISBN:1555811337 Relationships: is a type of GO:0031118